B cell proliferation [GO:0042100] (biological process) Also known as: B lymphocyte proliferation, B-cell proliferation, B-lymphocyte proliferation Subtypes: B cell proliferation involved in immune response [GO:0002322], GO:0002358, GO:0002359 Regulation: regulated by regulation of B cell proliferation [GO:0030888]; negatively regulated by negative regulation of B cell proliferation [GO:0030889]; positively regulated by positive regulation of B cell proliferation [GO:0030890] Sources: GOC:jl Relationships: is a type of B cell activation [GO:0042113]; is a type of lymphocyte proliferation [GO:0046651] Definition: The expansion of a B cell population by cell division. Follows B cell activation.